{
  "term_label": "Unknown biological process",
  "gene": "UniProtKB:Q0D2K5",
  "term_id": "UNKNOWN:0002",
  "gene_name": "Putative EGF-like and EMI domain-containing protein 1",
  "gene_symbol": "EGFEM1P"
}